anaerobic carbon tetrachloride metabolic process [GO:0018886] (biological process) Also known as: anaerobic carbon tetrachloride metabolism Sources: GOC:ai Definition: The chemical reactions and pathways involving carbon tetrachloride, a toxic, carcinogenic compound which is used as a general solvent in industrial degreasing operations, that occur in the absence of oxygen. Relationships: is a type of carbon tetrachloride metabolic process [GO:0018885]